sphingosine cholinephosphotransferase activity [GO:0047354] (molecular function) Relationships: is a type of phosphotransferase activity, for other substituted phosphate groups [GO:0016780] Definition: Catalysis of the reaction: CDP-choline + sphingosine = CMP + H+ + sphingosyl-phosphocholine. Sources: EC:2.7.8.10, RHEA:21224 Also known as: sphingosine choline phosphotransferase activity, CDP-choline-sphingosine cholinephosphotransferase activity, CDP-choline:sphingosine cholinephosphotransferase activity, cytidine diphosphocholine-sphingosine cholinephosphotransferase activity, phosphorylcholine-sphingosine transferase activity